{
  "term_label": "Unknown cellular component",
  "gene_symbol": "LGALS7",
  "gene_name": "Galectin-7",
  "term_id": "UNKNOWN:0003",
  "gene": "UniProtKB:P47929"
}